{
  "term_id": "GO:0016241",
  "gene_name": "Ubiquilin-1",
  "gene": "UniProtKB:Q9UMX0",
  "gene_symbol": "UBQLN1",
  "term_label": "regulation of macroautophagy"
}